{
  "term_id": "UNKNOWN:0002",
  "term_label": "Unknown biological process",
  "gene": "UniProtKB:Q9H777",
  "gene_name": "Zinc phosphodiesterase ELAC protein 1",
  "gene_symbol": "ELAC1"
}